{
  "gene_symbol": "CEP89",
  "term_id": "GO:0005814",
  "gene": "UniProtKB:Q96ST8",
  "gene_name": "Centrosomal protein of 89 kDa",
  "term_label": "centriole"
}